{
  "term_label": "intracellular zinc ion homeostasis",
  "gene_name": "Metallothionein 1H-like protein 1",
  "gene_symbol": "MT1HL1",
  "gene": "UniProtKB:P0DM35",
  "term_id": "GO:0006882"
}